{
  "gene": "UniProtKB:Q9NYA4",
  "gene_name": "Myotubularin-related protein 4",
  "term_label": "membrane",
  "term_id": "GO:0016020",
  "gene_symbol": "MTMR4"
}